myosin XVIII complex [GO:0031488] (cellular component) Definition: A myosin complex containing a class XVIII myosin heavy chain and associated light chains; myosin XVIII heavy chains contain an N-terminal PDZ domain. References: PMID:11294886 Relationships: is a type of unconventional myosin complex [GO:0016461]